{
  "gene": "UniProtKB:Q9H9A5",
  "term_label": "mRNA catabolic process",
  "gene_name": "CCR4-NOT transcription complex subunit 10",
  "term_id": "GO:0006402",
  "gene_symbol": "CNOT10"
}